{
  "term_id": "GO:0005813",
  "gene_name": "UPF0602 protein C4orf47",
  "gene_symbol": "C4orf47",
  "term_label": "centrosome",
  "gene": "UniProtKB:A7E2U8"
}